{
  "gene_name": "Cadherin-24",
  "gene": "UniProtKB:Q86UP0",
  "term_id": "GO:0008013",
  "gene_symbol": "CDH24",
  "term_label": "beta-catenin binding"
}